{
  "gene_name": "Protein tweety homolog 2",
  "gene_symbol": "TTYH2",
  "term_id": "GO:0005886",
  "gene": "UniProtKB:Q9BSA4",
  "term_label": "plasma membrane"
}